{
  "gene_symbol": "CRK",
  "term_id": "GO:0030971",
  "gene": "UniProtKB:P46108",
  "gene_name": "Adapter molecule crk",
  "term_label": "receptor tyrosine kinase binding"
}